{
  "gene": "UniProtKB:Q9HD67",
  "term_id": "GO:0005547",
  "gene_name": "Unconventional myosin-X",
  "term_label": "phosphatidylinositol-3,4,5-trisphosphate binding",
  "gene_symbol": "MYO10"
}